{
  "gene": "UniProtKB:A0AUZ9",
  "term_id": "GO:0035035",
  "gene_name": "KAT8 regulatory NSL complex subunit 1-like protein",
  "term_label": "histone acetyltransferase binding",
  "gene_symbol": "KANSL1L"
}